purine ribonucleoside bisphosphate catabolic process [GO:0034037] (biological process) Definition: The chemical reactions and pathways resulting in the breakdown of a purine ribonucleoside bisphosphate, a compound consisting of a purine base linked to a ribose sugar esterified with one phosphate group attached to each of two different hydroxyl groups on the sugar. Sources: GOC:mah, GOC:pde Also known as: purine ribonucleoside bisphosphate breakdown, purine ribonucleoside bisphosphate catabolism, purine ribonucleoside bisphosphate degradation Relationships: is a type of ribonucleoside bisphosphate catabolic process [GO:0034031]; is a type of GO:0034034; is a type of purine ribonucleoside bisphosphate metabolic process [GO:0034035] Subtypes: guanosine tetraphosphate catabolic process [GO:0015971], guanosine pentaphosphate catabolic process [GO:0015974]